snRNA modification guide activity [GO:0030566] (molecular function) References: PMID:12457565 Sources: GOC:mah Definition: Specifies the site of a posttranscriptional modification in an snRNA molecule by base pairing with a short sequence around the target residue. Note: Note that this term describes the activity of a nucleic acid, usually RNA, gene product that interacts with other RNA molecules via base pairing; it should not be used to annotate proteins. Relationships: is a type of snRNA binding [GO:0017069]; is a type of GO:0030555 Subtypes: snRNA 2'-O-ribose methylation guide activity [GO:0030563], snRNA pseudouridylation guide activity [GO:0030565]